{
  "term_label": "Unknown cellular component",
  "gene": "UniProtKB:Q6WQI6",
  "term_id": "UNKNOWN:0003",
  "gene_name": "Putative cancer susceptibility gene HEPN1 protein",
  "gene_symbol": "HEPN1"
}